{
  "term_label": "plasma membrane",
  "gene_name": "Olfactory receptor 6C70",
  "gene_symbol": "OR6C70",
  "term_id": "GO:0005886",
  "gene": "UniProtKB:A6NIJ9"
}